meiotic recombination nodule assembly [GO:0007146] (BP) Definition: During meiosis, the aggregation, arrangement and bonding together of strand exchange proteins (recombinases) to form small, electron dense structures in association with meiotic chromosomes. Subtypes: early meiotic recombination nodule assembly [GO:0042139], late meiotic recombination nodule assembly [GO:0042140] Relationships: is a type of meiotic DNA recombinase assembly [GO:0000707] References: PMID:9334324 Sources: GOC:jl